regulation of atrial cardiac muscle cell membrane depolarization [GO:0060371] (biological process) Relationships: is_a regulation of membrane depolarization [GO:0003254] Definition: Any process that modulates the establishment or extent of a membrane potential in the depolarizing direction away from the resting potential in an atrial cardiomyocyte. Sources: GOC:dph, GOC:tb Also known as: regulation of atrial cardiac muscle cell depolarization, regulation of atrial cardiomyocyte membrane depolarization, atrial depolarization, electrocardiogram PR interval